{
  "gene_name": "Microtubule-associated protein 1A",
  "term_id": "GO:0005875",
  "gene_symbol": "MAP1A",
  "gene": "UniProtKB:P78559",
  "term_label": "microtubule associated complex"
}